{
  "gene_symbol": "CLN3",
  "gene": "UniProtKB:Q13286",
  "term_id": "UNKNOWN:0001",
  "gene_name": "Battenin",
  "term_label": "Unknown molecular function"
}